negative regulation of nuclear migration during mitotic telophase [GO:1902853] (biological process) Relationships: is a type of negative regulation of nuclear migration along microtubule [GO:1902839]; is a type of regulation of nuclear migration during mitotic telophase [GO:1902852]; negatively regulates GO:0090561 Definition: Any process that stops, prevents or reduces the frequency, rate or extent of nuclear migration during mitotic telophase. References: PMID:23087209 Sources: GOC:TermGenie, GO_REF:0000058 Also known as: down regulation of nuclear migration during mitotic telophase, down-regulation of nuclear migration during mitotic telophase, downregulation of nuclear migration during mitotic telophase, inhibition of nuclear migration during mitotic telophase